{
  "gene_name": "Protein FAM117A",
  "gene_symbol": "FAM117A",
  "term_label": "Unknown molecular function",
  "term_id": "UNKNOWN:0001",
  "gene": "UniProtKB:Q9C073"
}